{
  "gene_symbol": "MYO5C",
  "gene": "UniProtKB:Q9NQX4",
  "gene_name": "Unconventional myosin-Vc",
  "term_label": "endocytosis",
  "term_id": "GO:0006897"
}